structural molecule activity conferring elasticity [GO:0097493] (molecular function) References: PMID:23283722 Sources: GOC:BHF, GOC:rl Subtypes: GO:0030023 Relationships: is a type of structural molecule activity [GO:0005198] Definition: The action of a molecule that contributes to the structural integrity of a complex or assembly within or outside a cell, providing elasticity and recoiling.